{
  "gene_symbol": "IGHV6-1",
  "term_id": "UNKNOWN:0003",
  "gene": "UniProtKB:A0A0B4J1U7",
  "term_label": "Unknown cellular component",
  "gene_name": "Immunoglobulin heavy variable 6-1"
}